cyclohexane-1,2-diol dehydrogenase activity [GO:0047795] (molecular function) Sources: EC:1.1.1.174, MetaCyc:CYCLOHEXANE-12-DIOL-DEHYDROGENASE-RXN Also known as: trans-cyclohexane-1,2-diol:NAD+ 1-oxidoreductase activity Definition: Catalysis of the reaction: trans-cyclohexane-1,2-diol + NAD+ = 2-hydroxycyclohexan-1-one + NADH. Relationships: is a type of oxidoreductase activity, acting on the CH-OH group of donors, NAD or NADP as acceptor [GO:0016616]